glycerophosphocholine cholinephosphodiesterase activity [GO:0047390] (molecular function) Also known as: L-3-glycerylphosphinicocholine cholinephosphohydrolase activity, sn-glycero-3-phosphocholine cholinephosphohydrolase activity Relationships: is a type of phosphoric diester hydrolase activity [GO:0008081] Definition: Catalysis of the reaction: sn-glycero-3-phosphocholine + H2O = choline phosphate + glycerol + H+. Sources: EC:3.1.4.38, RHEA:19545